pre-replicative complex [GO:0036387] (cellular component) Subtypes: GO:0005656, GO:0036389 Sources: GOC:bf, GOC:bhm, GOC:jh2, Wikipedia:Pre-replication_complex Definition: A protein-DNA complex that forms at the origin of replication during the initial step of DNA replication and allows the origin to become competent, or 'licensed', for replication. Relationships: is_a protein-DNA complex [GO:0032993] Also known as: pre-RC, pre-replication complex Note: This term describes pre-replicative complexes across organisms.